{
  "gene": "UniProtKB:Q9BT40",
  "term_label": "phosphatidylinositol-3,4,5-trisphosphate 5-phosphatase activity",
  "gene_name": "Inositol polyphosphate 5-phosphatase K",
  "term_id": "GO:0034485",
  "gene_symbol": "INPP5K"
}